{
  "gene": "UniProtKB:P43088",
  "gene_name": "Prostaglandin F2-alpha receptor",
  "term_label": "adenylate cyclase-activating G protein-coupled receptor signaling pathway",
  "gene_symbol": "PTGFR",
  "term_id": "GO:0007189"
}